{
  "term_id": "UNKNOWN:0002",
  "term_label": "Unknown biological process",
  "gene": "UniProtKB:A0A126GWI2",
  "gene_name": "Olfactory receptor",
  "gene_symbol": "OR2A25"
}